embryonic camera-type eye formation [GO:0060900] (biological process) Definition: The developmental process pertaining to the initial formation of a camera-type eye from unspecified neurectoderm. This process begins with the differentiation of cells that form the optic field and ends when the optic cup has attained its shape. Relationships: is a type of GO:0048646; is part of embryonic camera-type eye morphogenesis [GO:0048596] Sources: GOC:dph, GOC:sdb_2009, GOC:tb